viral release from host cell by cytolysis [GO:0044659] (biological process) Subtypes: GO:0039640, GO:0044660, viral release via disruption of host outer membrane [GO:0090680], viral release via disruption of host peptidoglycan cell wall [GO:0140913] Relationships: is a type of symbiont-mediated cytolysis of host cell [GO:0001897]; is a type of viral release from host cell [GO:0019076] References: PMID:26728778 Sources: GOC:jl Also known as: lytic viral release, viral exit from host cell by cytolysis, viral release by cell lysis, viral release by host cell lysis, cytolysis by virus of host cell, lytic viral life cycle Definition: The dissemination of mature viral particles from a host cell by the rupture of cell membranes and the loss of cytoplasm.